{
  "gene_name": "Scaffold attachment factor B2",
  "gene_symbol": "SAFB2",
  "gene": "UniProtKB:Q14151",
  "term_id": "GO:0005634",
  "term_label": "nucleus"
}